protein repair [GO:0030091] (biological process) Sources: GOC:mlg Definition: The process of restoring a protein to its original state after damage by such things as oxidation or spontaneous decomposition of residues. Subtypes: photosystem II repair [GO:0010206], protein deglycation [GO:0036525] Relationships: is_a protein metabolic process [GO:0019538]